sphingolipid delta-4 desaturase activity [GO:0042284] (molecular function) References: PMID:12417141 Sources: RHEA:46544 Definition: Catalysis of the reaction: an N-acylsphinganine + 2 Fe(II)-[cytochrome b5] + O2 + 2 H+ = an N-acylsphing-4-enine + 2 Fe(III)-[cytochrome b5] + 2 H2O. Also known as: delta-4 sphingolipid desaturase activity Relationships: is a type of GO:0016717